{
  "gene_symbol": "TPP1",
  "gene": "UniProtKB:O14773",
  "term_label": "tripeptidyl-peptidase activity",
  "gene_name": "Tripeptidyl-peptidase 1",
  "term_id": "GO:0008240"
}